regulation of imaginal disc-derived leg joint morphogenesis [GO:0110137] (biological process) References: PMID:25329825 Sources: GOC:ha Definition: Any process that modulates the frequency, rate or extent of imaginal disc-derived leg joint morphogenesis, the process in which the anatomical structure of the imaginal disc-derived leg joint is generated and organized. Relationships: is a type of GO:0022603; regulates GO:0007480 Subtypes: positive regulation of imaginal disc-derived leg joint morphogenesis [GO:0110138], negative regulation of imaginal disc-derived leg joint morphogenesis [GO:0110139]